positive regulation of phospholipid translocation [GO:0061092] (biological process) References: PMID:19966303 Sources: GOC:dph, GOC:jh, GOC:tb Definition: Any process that increases the frequency, rate or extent of the translocation, or flipping, of phospholipid molecules from one monolayer of a membrane bilayer to the opposite monolayer. Subtypes: positive regulation of phosphatidylserine exposure on apoptotic cell surface [GO:1905782] Relationships: is a type of positive regulation of cellular component organization [GO:0051130]; is a type of regulation of phospholipid translocation [GO:0061091]; is a type of positive regulation of phospholipid transport [GO:2001140]; positively regulates GO:0045332